{
  "term_id": "GO:0030027",
  "gene_name": "F-actin-uncapping protein LRRC16A",
  "gene": "UniProtKB:Q5VZK9",
  "gene_symbol": "CARMIL1",
  "term_label": "lamellipodium"
}